cardiac muscle myoblast proliferation [GO:0110021] (biological process) Relationships: is a type of myoblast proliferation [GO:0051450] Regulation: RO_0002211 by regulation of cardiac muscle myoblast proliferation [GO:0110022]; negatively regulated by negative regulation of cardiac muscle myoblast proliferation [GO:0110023]; positively regulated by GO:0110024 Definition: The multiplication or reproduction of cardiac muscle myoblasts, resulting in the expansion of a cardiac muscle myoblast cell population. A cardiac myoblast is a precursor cell that has been committed to a cardiac muscle cell fate but retains the ability to divide and proliferate throughout life. References: PMID:26512644 Sources: GOC:BHF, GOC:BHF_miRNA, GOC:rph